{
  "gene_symbol": "MEFV",
  "term_label": "cytosol",
  "term_id": "GO:0005829",
  "gene_name": "Pyrin",
  "gene": "UniProtKB:O15553"
}